{
  "term_id": "GO:0000183",
  "gene_name": "NAD-dependent protein deacetylase sirtuin-2",
  "term_label": "rDNA heterochromatin formation",
  "gene": "UniProtKB:Q8IXJ6",
  "gene_symbol": "SIRT2"
}